{
  "gene": "UniProtKB:Q9NY27",
  "gene_symbol": "PPP4R2",
  "term_label": "Unknown biological process",
  "term_id": "UNKNOWN:0002",
  "gene_name": "Serine_threonine-protein phosphatase 4 regulatory subunit 2"
}